{
  "gene_name": "Protection of telomeres protein 1",
  "term_id": "GO:0032210",
  "gene_symbol": "POT1",
  "term_label": "regulation of telomere maintenance via telomerase",
  "gene": "UniProtKB:Q9NUX5"
}